{
  "gene_name": "Myeloid zinc finger 1",
  "gene_symbol": "MZF1",
  "term_label": "DNA-binding transcription factor activity, RNA polymerase II-specific",
  "gene": "UniProtKB:P28698",
  "term_id": "GO:0000981"
}